negative regulation of axo-dendritic protein transport [GO:1905127] (biological process) Also known as: down regulation of axo-dendritic protein transport, down-regulation of axo-dendritic protein transport, downregulation of axo-dendritic protein transport, down regulation of axonal protein transport, down-regulation of axonal protein transport, downregulation of axonal protein transport, inhibition of axo-dendritic protein transport, inhibition of axonal protein transport, negative regulation of axonal protein transport Definition: Any process that stops, prevents or reduces the frequency, rate or extent of axo-dendritic protein transport. Relationships: is_a negative regulation of intracellular protein transport [GO:0090317]; is a type of regulation of axo-dendritic protein transport [GO:1905126]; negatively regulates axo-dendritic protein transport [GO:0099640] References: PMID:20694152 Sources: GOC:TermGenie, GO_REF:0000058